positive regulation of mannan catabolic process [GO:2000996] (biological process) Subtypes: positive regulation of glucomannan catabolic process [GO:2000908] Relationships: is a type of positive regulation of cell wall polysaccharide catabolic process [GO:2000968]; is a type of GO:2000994; RO_0002213 mannan catabolic process [GO:0046355] Also known as: positive regulation of mannan breakdown, positive regulation of mannan catabolism, positive regulation of mannan degradation Sources: GOC:mengo_curators Definition: Any process that activates or increases the frequency, rate or extent of mannan catabolic process.